{
  "gene": "UniProtKB:P18031",
  "gene_name": "Tyrosine-protein phosphatase non-receptor type 1",
  "term_id": "GO:1903898",
  "gene_symbol": "PTPN1",
  "term_label": "negative regulation of PERK-mediated unfolded protein response"
}